negative regulation of protein homotetramerization [GO:1901094] (biological process) Relationships: is_a negative regulation of protein homooligomerization [GO:0032463]; is a type of GO:1901091; is a type of regulation of protein homotetramerization [GO:1901093]; RO_0002212 GO:0051289 Also known as: down regulation of protein homotetramer assembly, down regulation of protein homotetramer biosynthesis, down regulation of protein homotetramer biosynthetic process, down regulation of protein homotetramer formation, down regulation of protein homotetramerization, down-regulation of protein homotetramer assembly, down-regulation of protein homotetramer biosynthesis, down-regulation of protein homotetramer biosynthetic process, down-regulation of protein homotetramer formation, down-regulation of protein homotetramerization, downregulation of protein homotetramer assembly, downregulation of protein homotetramer biosynthesis, downregulation of protein homotetramer biosynthetic process, downregulation of protein homotetramer formation, downregulation of protein homotetramerization, negative regulation of protein homotetramer assembly, negative regulation of protein homotetramer biosynthesis, negative regulation of protein homotetramer biosynthetic process, negative regulation of protein homotetramer formation, inhibition of protein homotetramer assembly, inhibition of protein homotetramer biosynthesis, inhibition of protein homotetramer biosynthetic process, inhibition of protein homotetramer formation, inhibition of protein homotetramerization Definition: Any process that stops, prevents or reduces the frequency, rate or extent of protein homotetramerization. Sources: GOC:TermGenie, GOC:pm